{
  "gene": "UniProtKB:Q9P0U3",
  "gene_name": "Sentrin-specific protease 1",
  "term_id": "GO:0016926",
  "gene_symbol": "SENP1",
  "term_label": "protein desumoylation"
}